xanthophyll cycle [GO:0010028] (biological process) Sources: ISBN:0122146743 Definition: A cyclic series of interconversions involving three xanthophylls, violoxanthin, antheraxanthin, and zeaxanthin. The xanthophyll cycle is involved in regulating energy dissipation in light harvesting complex II. Relationships: is a type of xanthophyll metabolic process [GO:0016122]